{
  "gene_symbol": "ACVRL1",
  "term_id": "GO:0030509",
  "term_label": "BMP signaling pathway",
  "gene": "UniProtKB:P37023",
  "gene_name": "Serine_threonine-protein kinase receptor R3"
}